{
  "term_label": "Unknown molecular function",
  "gene_name": "Proton-activated chloride channel",
  "term_id": "UNKNOWN:0001",
  "gene_symbol": "PACC1",
  "gene": "UniProtKB:Q9H813"
}